{
  "gene": "UniProtKB:Q9Y3Y2",
  "term_label": "chromatin remodeling",
  "gene_name": "Chromatin target of PRMT1 protein",
  "term_id": "GO:0006338",
  "gene_symbol": "CHTOP"
}